{
  "gene_name": "Keratin, type II cytoskeletal 7",
  "gene": "UniProtKB:P08729",
  "term_label": "structural constituent of skin epidermis",
  "term_id": "GO:0030280",
  "gene_symbol": "KRT7"
}